{
  "term_id": "GO:0043235",
  "gene_symbol": "MUSK",
  "gene": "UniProtKB:O15146",
  "term_label": "receptor complex",
  "gene_name": "Muscle, skeletal receptor tyrosine-protein kinase"
}